{
  "term_label": "ERAD pathway",
  "gene_name": "Calmegin",
  "gene_symbol": "CLGN",
  "gene": "UniProtKB:O14967",
  "term_id": "GO:0036503"
}